{
  "gene": "UniProtKB:P50151",
  "term_label": "G-protein beta-subunit binding",
  "term_id": "GO:0031681",
  "gene_name": "Guanine nucleotide-binding protein G(I)_G(S)_G(O) subunit gamma-10",
  "gene_symbol": "GNG10"
}